{
  "term_id": "GO:0008284",
  "gene_symbol": "CNTFR",
  "gene_name": "Ciliary neurotrophic factor receptor subunit alpha",
  "gene": "UniProtKB:P26992",
  "term_label": "positive regulation of cell population proliferation"
}